{
  "gene_name": "Taste receptor type 2 member 45",
  "gene_symbol": "TAS2R45",
  "gene": "UniProtKB:P59539",
  "term_id": "UNKNOWN:0001",
  "term_label": "Unknown molecular function"
}